{
  "gene": "UniProtKB:Q5HYM0",
  "term_id": "GO:0003729",
  "gene_symbol": "ZC3H12B",
  "term_label": "mRNA binding",
  "gene_name": "Probable ribonuclease ZC3H12B"
}